proline dipeptidase activity [GO:0102009] (MF) Relationships: is a type of dipeptidase activity [GO:0016805] Definition: Catalysis of the reaction: H2O + a dipeptide with proline at the C-terminal = L-proline + a standard alpha amino acid. Sources: EC:3.4.13.9